{
  "term_label": "guanyl-nucleotide exchange factor activity",
  "gene": "UniProtKB:Q0VGL1",
  "gene_symbol": "LAMTOR4",
  "gene_name": "Ragulator complex protein LAMTOR4",
  "term_id": "GO:0005085"
}